{
  "gene_symbol": "MAP2K6",
  "term_id": "UNKNOWN:0003",
  "gene": "UniProtKB:P52564",
  "term_label": "Unknown cellular component",
  "gene_name": "Dual specificity mitogen-activated protein kinase kinase 6"
}